{
  "gene_symbol": "RAB24",
  "term_label": "GTPase activity",
  "gene_name": "Ras-related protein Rab-24",
  "term_id": "GO:0003924",
  "gene": "UniProtKB:Q969Q5"
}